{
  "term_label": "nucleus",
  "gene": "UniProtKB:O60927",
  "gene_symbol": "PPP1R11",
  "gene_name": "E3 ubiquitin-protein ligase PPP1R11",
  "term_id": "GO:0005634"
}